{
  "term_label": "RNA binding",
  "gene_name": "ATP-dependent RNA helicase A",
  "term_id": "GO:0003723",
  "gene_symbol": "DHX9",
  "gene": "UniProtKB:Q08211"
}